{
  "term_id": "GO:0005783",
  "gene": "UniProtKB:Q9NXF8",
  "gene_name": "Palmitoyltransferase ZDHHC7",
  "gene_symbol": "ZDHHC7",
  "term_label": "endoplasmic reticulum"
}